{
  "gene_symbol": "FBXW9",
  "term_id": "UNKNOWN:0001",
  "gene_name": "F-box_WD repeat-containing protein 9",
  "term_label": "Unknown molecular function",
  "gene": "UniProtKB:Q5XUX1"
}